{
  "gene_name": "tRNA N6-adenosine threonylcarbamoyltransferase",
  "gene_symbol": "OSGEP",
  "term_label": "EKC/KEOPS complex",
  "gene": "UniProtKB:Q9NPF4",
  "term_id": "GO:0000408"
}